{
  "gene": "UniProtKB:P32119",
  "term_id": "GO:0008379",
  "gene_name": "Peroxiredoxin-2",
  "gene_symbol": "PRDX2",
  "term_label": "thioredoxin peroxidase activity"
}